{
  "gene_name": "Serine palmitoyltransferase 1",
  "term_label": "serine C-palmitoyltransferase activity",
  "term_id": "GO:0004758",
  "gene_symbol": "SPTLC1",
  "gene": "UniProtKB:O15269"
}